pseudopodium retraction [GO:0031270] (biological process) Sources: GOC:pg Definition: The myosin-based contraction and retraction of a pseudopodium. Relationships: is a type of cellular component disassembly [GO:0022411]; is a type of pseudopodium organization [GO:0031268] Subtypes: lateral pseudopodium retraction [GO:0120320]